{
  "term_id": "GO:0005615",
  "gene": "UniProtKB:O14793",
  "term_label": "extracellular space",
  "gene_name": "Growth_differentiation factor 8",
  "gene_symbol": "MSTN"
}